synaptobrevin 2-SNAP-25-syntaxin-1a complex [GO:0070044] (CC) Relationships: is a type of SNARE complex [GO:0031201] Definition: A SNARE complex that contains synaptobrevin 2 (VAMP2), SNAP-25, and syntaxin 1a (or orthologs thereof). Also known as: SNARE complex (Snap25, Stx1a, Vamp2), SNARE complex (Stx1a, SNAP25, VAMP), Snap25-Stx1a-Vamp2 complex, Stx1a-SNAP25-VAMP complex References: PMID:10336434